{
  "gene": "UniProtKB:P32248",
  "term_label": "immune response",
  "gene_name": "C-C chemokine receptor type 7",
  "term_id": "GO:0006955",
  "gene_symbol": "CCR7"
}